spectrin-associated cytoskeleton [GO:0014731] (cellular component) References: PMID:15970557 Sources: GOC:mtg_muscle Relationships: is a type of cytoskeleton [GO:0005856] Subtypes: postsynaptic spectrin-associated cytoskeleton [GO:0099189] Definition: The part of the cytoskeleton composed of spectrin, protein 4.1 and ankyrin. Spectrin-associated cytoskeleton is associated with the plasma membrane.